{
  "gene": "UniProtKB:P50225",
  "term_label": "aryl sulfotransferase activity",
  "gene_name": "Sulfotransferase 1A1",
  "gene_symbol": "SULT1A1",
  "term_id": "GO:0004062"
}